{
  "gene": "UniProtKB:O43716",
  "term_id": "GO:0005739",
  "gene_name": "Glutamyl-tRNA(Gln) amidotransferase subunit C, mitochondrial",
  "term_label": "mitochondrion",
  "gene_symbol": "GATC"
}